{
  "gene_name": "Insulin-like growth factor-binding protein 4",
  "term_label": "insulin-like growth factor I binding",
  "term_id": "GO:0031994",
  "gene": "UniProtKB:P22692",
  "gene_symbol": "IGFBP4"
}